cleavage furrow formation [GO:0036089] (biological process) Also known as: cleavage furrow positioning Relationships: is a type of GO:0032506; is a type of plasma membrane invagination [GO:0099024]; is part of cytoskeleton-dependent cytokinesis [GO:0061640] Note: Consider also annotating to 'establishment of contractile ring localization involved in cell cycle cytokinesis ; GO:0032188'. Subtypes: mitotic cleavage furrow formation [GO:1903673] Definition: Generation of the cleavage furrow, a shallow groove in the cell surface near the old metaphase plate that marks the site of cytokinesis. This process includes the recruitment and localized activation of signals such as RhoA at the site of the future furrow to ensure that furrowing initiates at the correct site in the cell. References: PMID:15811947, PMID:20687468, PMID:2192590 Sources: GOC:ans